{
  "term_label": "Cul4-RING E3 ubiquitin ligase complex",
  "term_id": "GO:0080008",
  "gene": "UniProtKB:Q9Y4B6",
  "gene_symbol": "DCAF1",
  "gene_name": "DDB1- and CUL4-associated factor 1"
}